positive regulation of post-transcriptional gene silencing [GO:0060148] (biological process) Sources: GOC:dph Subtypes: positive regulation of post-transcriptional gene silencing by RNA [GO:1900370] Also known as: positive regulation of posttranscriptional gene silencing Definition: Any process that increases the frequency, rate or extent of the inactivation of gene expression by a posttranscriptional mechanism. Relationships: is a type of GO:0048518; is a type of regulation of post-transcriptional gene silencing [GO:0060147]; positively regulates post-transcriptional gene silencing [GO:0016441]